{
  "term_id": "GO:0005634",
  "gene": "UniProtKB:Q16236",
  "gene_name": "Nuclear factor erythroid 2-related factor 2",
  "term_label": "nucleus",
  "gene_symbol": "NFE2L2"
}